response to host pH environment [GO:0075293] (biological process) Also known as: response of symbiont to host pH environment Definition: Any process that results in a change in state or activity of the symbiont or its cell (in terms of movement, secretion, enzyme production, gene expression, etc.) as a result of the pH conditions in or around its host organism. The host is defined as the larger of the organisms involved in a symbiotic interaction. Relationships: is a type of response to host [GO:0075136] Sources: GOC:pamgo_curators